{
  "gene_symbol": "ZSCAN9",
  "term_label": "regulation of transcription by RNA polymerase II",
  "term_id": "GO:0006357",
  "gene": "UniProtKB:O15535",
  "gene_name": "Zinc finger and SCAN domain-containing protein 9"
}